protein-DNA ISRE complex [GO:0097522] (cellular component) References: PMID:11747630 Sources: GOC:amm, GOC:cjm Definition: A protein-DNA complex formed through interaction of the protein(s) with an interferon-stimulated response element (ISRE) in the DNA. Relationships: is a type of protein-DNA complex [GO:0032993]